{
  "gene": "UniProtKB:Q9Y5E8",
  "term_id": "GO:0005886",
  "gene_name": "Protocadherin beta-15",
  "term_label": "plasma membrane",
  "gene_symbol": "PCDHB15"
}